{
  "gene_symbol": "PDE6B",
  "gene": "UniProtKB:P35913",
  "term_id": "GO:0042622",
  "term_label": "photoreceptor outer segment membrane",
  "gene_name": "Rod cGMP-specific 3',5'-cyclic phosphodiesterase subunit beta"
}